{
  "term_label": "protein serine/threonine kinase activity",
  "term_id": "GO:0004674",
  "gene_name": "Mitogen-activated protein kinase kinase kinase 20",
  "gene_symbol": "MAP3K20",
  "gene": "UniProtKB:Q9NYL2"
}